4-hydroxysphinganine ceramide fatty acyl 2-hydroxylase activity [GO:0120521] (molecular function) Definition: Catalysis of the reaction: an N-(1,2 saturated acyl)-(4R)-hydroxysphinganine + 2 Fe(II)-[cytochrome b5] + 2 H+ + O2 = an N-(2R-hydroxyacyl)-4R-hydroxysphinganine + 2 Fe(III)-[cytochrome b5] + H2O. Relationships: is a type of GO:0080132 Sources: RHEA:46520